{
  "term_label": "positive regulation of T cell mediated cytotoxicity",
  "gene_name": "T-cell surface glycoprotein CD1a",
  "gene_symbol": "CD1A",
  "term_id": "GO:0001916",
  "gene": "UniProtKB:P06126"
}